{
  "term_id": "GO:0006597",
  "gene_symbol": "AMD1",
  "term_label": "spermine biosynthetic process",
  "gene_name": "S-adenosylmethionine decarboxylase proenzyme",
  "gene": "UniProtKB:P17707"
}